{
  "gene_symbol": "GPR15L",
  "term_label": "extracellular region",
  "gene": "UniProtKB:Q6UWK7",
  "gene_name": "Protein GPR15LG",
  "term_id": "GO:0005576"
}